{
  "gene_name": "Cyclic nucleotide-gated cation channel beta-3",
  "term_label": "intracellular cyclic nucleotide activated cation channel complex",
  "term_id": "GO:0017071",
  "gene": "UniProtKB:Q9NQW8",
  "gene_symbol": "CNGB3"
}